{
  "gene_symbol": "ARMC8",
  "term_label": "proteasome-mediated ubiquitin-dependent protein catabolic process",
  "gene": "UniProtKB:Q8IUR7",
  "gene_name": "Armadillo repeat-containing protein 8",
  "term_id": "GO:0043161"
}